{
  "gene_symbol": "IL4R",
  "gene_name": "Interleukin-4 receptor subunit alpha",
  "term_label": "interleukin-4-mediated signaling pathway",
  "term_id": "GO:0035771",
  "gene": "UniProtKB:P24394"
}